negative regulation of short-term neuronal synaptic plasticity [GO:0048174] (biological process) References: PMID:11891290 Sources: GOC:jid Relationships: is a type of regulation of short-term neuronal synaptic plasticity [GO:0048172]; is a type of GO:0050768 Note: Note that the syntax of the definition of this term is different from the usual regulation syntax because it describes regulation of a trait rather than regulation of a process. Definition: A process that decreases short-term neuronal synaptic plasticity, the ability of neuronal synapses to change in the short-term as circumstances require. Short-term neuronal synaptic plasticity generally involves increasing or decreasing synaptic sensitivity. Also known as: down regulation of short-term neuronal synaptic plasticity, down-regulation of short-term neuronal synaptic plasticity, downregulation of short-term neuronal synaptic plasticity, inhibition of short-term neuronal synaptic plasticity